protein-phosphocysteine-L-ascorbate-phosphotransferase system transporter activity [GO:0090585] (molecular function) References: PMID:15153772 Definition: Catalysis of the PEP-dependent, phosphoryl transfer-driven transport of substances across a membrane. The transport happens by catalysis of the reaction: protein S-phosphocysteine + L-ascorbate(out) = protein cysteine + L-ascorbate-6-phosphate(in). Relationships: is a type of protein-phosphocysteine-sugar phosphotransferase activity [GO:0090563]